{
  "gene_name": "Membrane frizzled-related protein",
  "term_id": "UNKNOWN:0002",
  "term_label": "Unknown biological process",
  "gene": "UniProtKB:Q9BY79",
  "gene_symbol": "MFRP"
}